{
  "term_label": "Unknown biological process",
  "gene_name": "Dihydropyrimidinase-related protein 4",
  "gene_symbol": "DPYSL4",
  "gene": "UniProtKB:O14531",
  "term_id": "UNKNOWN:0002"
}